{
  "gene_symbol": "ZNF571",
  "term_id": "GO:0000978",
  "gene": "UniProtKB:Q7Z3V5",
  "gene_name": "Zinc finger protein 571",
  "term_label": "RNA polymerase II cis-regulatory region sequence-specific DNA binding"
}